{
  "term_id": "GO:0005172",
  "gene_name": "Placenta growth factor",
  "term_label": "vascular endothelial growth factor receptor binding",
  "gene": "UniProtKB:P49763",
  "gene_symbol": "PGF"
}